{
  "gene": "UniProtKB:Q96N77",
  "term_label": "DNA-binding transcription factor activity, RNA polymerase II-specific",
  "gene_symbol": "ZNF641",
  "gene_name": "Zinc finger protein 641",
  "term_id": "GO:0000981"
}